{
  "gene_name": "Homeobox protein Hox-A6",
  "gene_symbol": "HOXA6",
  "term_label": "anterior/posterior pattern specification",
  "gene": "UniProtKB:P31267",
  "term_id": "GO:0009952"
}